{
  "term_label": "positive regulation of cytosolic calcium ion concentration",
  "term_id": "GO:0007204",
  "gene_symbol": "FPR3",
  "gene": "UniProtKB:P25089",
  "gene_name": "N-formyl peptide receptor 3"
}